{
  "term_id": "GO:0000976",
  "term_label": "transcription cis-regulatory region binding",
  "gene": "UniProtKB:Q6ZN19",
  "gene_symbol": "ZNF841",
  "gene_name": "Zinc finger protein 841"
}